{
  "term_label": "microtubule cytoskeleton",
  "gene": "UniProtKB:Q9H7U1",
  "gene_name": "Serine-rich coiled-coil domain-containing protein 2",
  "gene_symbol": "CCSER2",
  "term_id": "GO:0015630"
}